erythronolide synthase activity [GO:0047879] (molecular function) Definition: Catalysis of the reaction: 6 malonyl-CoA + propionyl-CoA = 7 CoA + 6-deoxyerythronolide B. Also known as: erythronolide condensing enzyme activity, malonyl-CoA:propionyl-CoA malonyltransferase (cyclizing) Relationships: is a type of GO:0016747 Sources: EC:2.3.1.94, MetaCyc:ERYTHRONOLIDE-SYNTHASE-RXN